{
  "gene_symbol": "NAA50",
  "term_label": "protein-lysine-acetyltransferase activity",
  "gene": "UniProtKB:Q9GZZ1",
  "gene_name": "N-alpha-acetyltransferase 50",
  "term_id": "GO:0061733"
}